{
  "term_label": "outward rectifier potassium channel activity",
  "gene_symbol": "KCNK3",
  "gene": "UniProtKB:O14649",
  "term_id": "GO:0015271",
  "gene_name": "Potassium channel subfamily K member 3"
}